mitochondrial protein-containing complex [GO:0098798] (cellular component) Subtypes: mitochondrial creatine kinase complex [GO:0002187], mitochondrial permeability transition pore complex [GO:0005757], GO:0005760, mitochondrial large ribosomal subunit [GO:0005762], GO:0005763, mitochondrial endopeptidase Clp complex [GO:0009841], mitochondrial fatty acid beta-oxidation multienzyme complex [GO:0016507], mitochondrial processing peptidase complex [GO:0017087], mitochondrial electron transfer flavoprotein complex [GO:0017133], mitochondrial pyruvate dehydrogenase (lipoamide) phosphatase complex [GO:0019910], GO:0030678, mitochondrial mRNA editing complex [GO:0031019], mitochondrial DNA-directed RNA polymerase complex [GO:0034245], Ecsit-NDUFAF1 complex [GO:0034985], mitochondrial intermembrane space chaperone complex [GO:0042719], mitochondrial glutamate synthase complex (NADH) [GO:0043294], mitochondrial degradosome [GO:0045025], GO:0061671, outer mitochondrial membrane protein complex [GO:0098799], inner mitochondrial membrane protein complex [GO:0098800], mitochondrial [2Fe-2S] assembly complex [GO:0099128], GO:0106098, GO:0120510, mitochondrial translation initiation complex [GO:0180052], mitochondrial translation preinitiation complex [GO:0180053] Relationships: is a type of GO:0032991; is part of mitochondrion [GO:0005739] Note: Note that this term is in the subset of terms that should not be used for direct gene product annotation. Instead, select a child term or, if no appropriate child term exists, please request a new term. Direct annotations to this term may be amended during annotation QC. Sources: GOC:dos Also known as: mitochondrial protein complex Definition: A protein complex that is part of a mitochondrion.